{
  "gene": "UniProtKB:O95201",
  "term_id": "GO:0006357",
  "gene_symbol": "ZNF205",
  "term_label": "regulation of transcription by RNA polymerase II",
  "gene_name": "Transcriptional repressor RHIT"
}